glycosome [GO:0020015] (cellular component) Definition: A membrane-bounded organelle found in organisms from the order Kinetoplastida that houses the enzymes of glycolysis. Sources: GOC:mb Relationships: is a type of peroxisome [GO:0005777]